{
  "gene": "UniProtKB:Q9H0A8",
  "gene_symbol": "COMMD4",
  "term_label": "signal transduction",
  "term_id": "GO:0007165",
  "gene_name": "COMM domain-containing protein 4"
}